{
  "gene_name": "Macrosialin",
  "gene_symbol": "CD68",
  "term_id": "GO:0005765",
  "gene": "UniProtKB:P34810",
  "term_label": "lysosomal membrane"
}